{
  "term_label": "synaptic transmission, glycinergic",
  "term_id": "GO:0060012",
  "gene_symbol": "SLC6A5",
  "gene": "UniProtKB:Q9Y345",
  "gene_name": "Sodium- and chloride-dependent glycine transporter 2"
}